{
  "gene_name": "Olfactory receptor 9I1",
  "gene": "UniProtKB:Q8NGQ6",
  "term_label": "G protein-coupled receptor signaling pathway",
  "term_id": "GO:0007186",
  "gene_symbol": "OR9I1"
}